{
  "gene": "UniProtKB:O60806",
  "term_label": "heart morphogenesis",
  "gene_symbol": "TBX19",
  "gene_name": "T-box transcription factor TBX19",
  "term_id": "GO:0003007"
}